{
  "term_id": "GO:0016255",
  "gene": "UniProtKB:Q969N2",
  "gene_symbol": "PIGT",
  "term_label": "attachment of GPI anchor to protein",
  "gene_name": "GPI transamidase component PIG-T"
}